{
  "gene_symbol": "ZNF555",
  "gene_name": "Zinc finger protein 555",
  "term_label": "regulation of transcription by RNA polymerase II",
  "term_id": "GO:0006357",
  "gene": "UniProtKB:Q8NEP9"
}